interleukin-26 receptor binding [GO:0045522] (molecular function) Sources: GOC:go_curators Definition: Binding to an interleukin-26 receptor. Also known as: IL-26, interleukin-26 receptor ligand Relationships: is a type of GO:0005126